{
  "term_label": "semaphorin receptor complex",
  "term_id": "GO:0002116",
  "gene_symbol": "PLXNA2",
  "gene_name": "Plexin-A2",
  "gene": "UniProtKB:O75051"
}